{
  "gene": "UniProtKB:P25100",
  "term_id": "GO:0045907",
  "term_label": "positive regulation of vasoconstriction",
  "gene_symbol": "ADRA1D",
  "gene_name": "Alpha-1D adrenergic receptor"
}